positive regulation of microtubule polymerization or depolymerization [GO:0031112] (biological process) Subtypes: positive regulation of microtubule polymerization [GO:0031116], positive regulation of microtubule depolymerization [GO:0031117] Definition: Any process that activates or increases the frequency, rate or extent of microtubule polymerization or depolymerization. Also known as: up regulation of microtubule polymerization or depolymerization, up-regulation of microtubule polymerization or depolymerization, upregulation of microtubule polymerization or depolymerization, activation of microtubule polymerization or depolymerization, stimulation of microtubule polymerization or depolymerization Sources: GOC:mah Relationships: is a type of regulation of microtubule polymerization or depolymerization [GO:0031110]; is a type of GO:0051495; positively regulates microtubule polymerization or depolymerization [GO:0031109]